{
  "term_label": "cytosol",
  "gene": "UniProtKB:Q9Y6M1",
  "gene_name": "Insulin-like growth factor 2 mRNA-binding protein 2",
  "term_id": "GO:0005829",
  "gene_symbol": "IGF2BP2"
}